regulation of androstenedione secretion [GO:2000837] (biological process) Also known as: regulation of androst-4-ene-3,17-dione secretion Relationships: is a type of regulation of lipid transport [GO:0032368]; is a type of GO:0046883; regulates androstenedione secretion [GO:0035941] Sources: GOC:sl Subtypes: negative regulation of androstenedione secretion [GO:2000838], GO:2000839 Definition: Any process that modulates the frequency, rate or extent of androstenedione secretion.